{
  "term_id": "UNKNOWN:0002",
  "gene_name": "Aldo-keto reductase family 1 member A1",
  "gene": "UniProtKB:P14550",
  "term_label": "Unknown biological process",
  "gene_symbol": "AKR1A1"
}